{
  "gene_name": "Ankyrin repeat domain-containing protein SOWAHD",
  "term_id": "UNKNOWN:0001",
  "gene_symbol": "SOWAHD",
  "term_label": "Unknown molecular function",
  "gene": "UniProtKB:A6NJG2"
}